D-alanine import across plasma membrane [GO:0170048] (biological process) Relationships: is a type of GO:0042941 References: PMID:22418438, PMID:25425233 Also known as: D-alanine import, D-alanine import into cell, D-alanine uptake Definition: The directed import of D-alanine from the extracellular region across the plasma membrane and into the cytosol.